{
  "gene": "UniProtKB:P59037",
  "term_id": "UNKNOWN:0002",
  "gene_symbol": "LINC00313",
  "term_label": "Unknown biological process",
  "gene_name": "Putative uncharacterized protein encoded by LINC00313"
}